paraflagellar rod assembly [GO:0120268] (biological process) Also known as: paraflagellar rod biogenesis, paraflagellar rod formation, PFR assembly Definition: The aggregation, arrangement and bonding together of a set of components to form a paraflagellar rod, a large lattice-like axial structure found in some flagellated protists which extends alongside the axoneme. Relationships: is a type of motile cilium assembly [GO:0044458] References: PMID:23787017, PMID:32295845 Sources: GOC:ach, GOC:krc